{
  "gene_name": "U2 small nuclear ribonucleoprotein auxiliary factor 35 kDa subunit-related protein 2",
  "term_label": "U2AF complex",
  "gene_symbol": "ZRSR2",
  "term_id": "GO:0089701",
  "gene": "UniProtKB:Q15696"
}